alkan-1-ol dehydrogenase (acceptor) activity [GO:0047645] (molecular function) Also known as: polyethylene glycol dehydrogenase activity, alkan-1-ol:(acceptor) oxidoreductase activity, alkan-1-ol:acceptor oxidoreductase activity Definition: Catalysis of the reaction: primary alcohol + acceptor = aldehyde + reduced acceptor. Relationships: is a type of oxidoreductase activity, acting on CH-OH group of donors [GO:0016614] Sources: EC:1.1.99.20, MetaCyc:ALKAN-1-OL-DEHYDROGENASE-ACCEPTOR-RXN